{
  "term_id": "GO:0032438",
  "term_label": "melanosome organization",
  "gene_symbol": "GPR143",
  "gene": "UniProtKB:P51810",
  "gene_name": "G-protein coupled receptor 143"
}